{
  "gene_symbol": "GTF2H3",
  "gene": "UniProtKB:Q13889",
  "term_label": "transcription factor TFIIH holo complex",
  "term_id": "GO:0005675",
  "gene_name": "General transcription factor IIH subunit 3"
}